{
  "term_id": "UNKNOWN:0001",
  "gene_name": "Podocan-like protein 1",
  "term_label": "Unknown molecular function",
  "gene_symbol": "PODNL1",
  "gene": "UniProtKB:Q6PEZ8"
}